establishment of imaginal disc-derived wing hair orientation [GO:0001737] (BP) References: PMID:11239465 Sources: GOC:ascb_2009, GOC:dph, GOC:mtg_sensu, GOC:tb Also known as: establishment of wing hair orientation Definition: Orientation of hairs in the imaginal disc-derived wing along a proximal-distal axis, such that each cell of the wing produces one wing hair which points in a distal direction. Relationships: is a type of establishment of planar polarity [GO:0001736]; is a type of post-embryonic animal morphogenesis [GO:0009886]; BFO_0000050 imaginal disc-derived wing hair organization [GO:0035317]